regulation of norepinephrine secretion [GO:0014061] (biological process) Definition: Any process that modulates the frequency, rate or extent of the regulated release of norepinephrine. Also known as: regulation of noradrenaline secretion Relationships: is a type of GO:0050433; regulates norepinephrine secretion [GO:0048243] Sources: GOC:ef Subtypes: GO:0010700, positive regulation of norepinephrine secretion [GO:0010701]